{
  "term_label": "P granule",
  "gene_name": "Piwi-like protein 4",
  "term_id": "GO:0043186",
  "gene_symbol": "PIWIL4",
  "gene": "UniProtKB:Q7Z3Z4"
}